neutrophil-mediated killing of gram-positive bacterium [GO:0070946] (biological process) Relationships: is a type of neutrophil-mediated killing of bacterium [GO:0070944]; is part of defense response to Gram-positive bacterium [GO:0050830] Regulation: RO_0002211 by regulation of neutrophil mediated killing of gram-positive bacterium [GO:0070952]; negatively regulated by negative regulation of neutrophil mediated killing of gram-positive bacterium [GO:0070958]; RO_0002213 by positive regulation of neutrophil mediated killing of gram-positive bacterium [GO:0070964] Also known as: neutrophil mediated killing of gram-positive bacterium Definition: The directed killing of a gram-positive bacterium by a neutrophil. Sources: GOC:add, ISBN:0781765196